GDP-mannose pyrophosphorylase complex [GO:0120508] (cellular component) Relationships: is a type of transferase complex, transferring phosphorus-containing groups [GO:0061695] Definition: A protein complex capable of catalyzing the reaction of GTP and mannose-1-phosphate to form GDP-mannose. The complex is a homodimer in most bacteria and a heterodimer in most eukaryotes. In humans, it is composed of a catalytic beta subunit (GMPPB) and a regulatory alpha subunit (GMPPA). Also known as: GMPPA-GMPPB complex References: PMID:33986552 Sources: GOC:sjm